{
  "gene_name": "Dual specificity protein kinase CLK3",
  "term_label": "protein serine/threonine kinase activity",
  "term_id": "GO:0004674",
  "gene": "UniProtKB:P49761",
  "gene_symbol": "CLK3"
}